G protein-coupled GABA receptor complex [GO:1902712] (cellular component) Definition: A protein complex which is capable of G protein-coupled GABA receptor activity. In human, it is usually a heterodimer composed of GABA-B receptor subunits 1 and 2. References: PMID:18790874 Sources: GOC:TermGenie, GOC:bhm, GO_REF:0000088 Also known as: G-protein coupled GABA receptor complex Relationships: is a type of GO:0038037; is a type of GABA receptor complex [GO:1902710] Note: An example of this is GABR1 in human (UniProt symbol Q9UBS5) in PMID:18790874.